{
  "gene": "UniProtKB:P04150",
  "gene_symbol": "NR3C1",
  "term_label": "estrogen response element binding",
  "gene_name": "Glucocorticoid receptor",
  "term_id": "GO:0034056"
}